{
  "gene_name": "Endoplasmic reticulum-Golgi intermediate compartment protein 1",
  "gene_symbol": "ERGIC1",
  "term_label": "endoplasmic reticulum to Golgi vesicle-mediated transport",
  "gene": "UniProtKB:Q969X5",
  "term_id": "GO:0006888"
}